{
  "term_label": "Unknown biological process",
  "gene": "UniProtKB:Q71RG6",
  "gene_symbol": "FP248",
  "term_id": "UNKNOWN:0002",
  "gene_name": "Putative chemokine-related protein FP248"
}